{
  "gene_symbol": "CHMP4C",
  "term_id": "GO:0006900",
  "gene": "UniProtKB:Q96CF2",
  "gene_name": "Charged multivesicular body protein 4c",
  "term_label": "vesicle budding from membrane"
}